primary thickening [GO:0080192] (biological process) Relationships: is a type of GO:0080190 Sources: ISBN:0471245208, JSTOR:4354165, PO:0005039, PO:0025004 Note: Occurs in shoot axes and rarely in roots in many monocotyledons. Definition: Lateral growth of a plant axis (shoot axis or root) that is an increase in thickness resulting from the activity of a primary thickening meristem.